{
  "gene": "UniProtKB:Q53EV4",
  "term_id": "GO:0005829",
  "gene_symbol": "LRRC23",
  "term_label": "cytosol",
  "gene_name": "Leucine-rich repeat-containing protein 23"
}